{
  "term_id": "GO:0005543",
  "gene": "UniProtKB:P02656",
  "gene_name": "Apolipoprotein C-III",
  "term_label": "phospholipid binding",
  "gene_symbol": "APOC3"
}